{
  "term_label": "mRNA 3'-UTR binding",
  "gene_name": "Deleted in azoospermia protein 2",
  "gene": "UniProtKB:Q13117",
  "term_id": "GO:0003730",
  "gene_symbol": "DAZ2"
}